seed coat development [GO:0010214] (biological process) Definition: The process whose specific outcome is the progression of the seed coat over time, from its formation to the mature structure. Relationships: is a type of developmental process involved in reproduction [GO:0003006]; is a type of GO:0048856; is part of GO:0048316 Sources: GOC:go_curators